S-adenosyl-L-methionine binding [GO:1904047] (molecular function) Also known as: radical SAM enzyme activity References: PMID:22985361 Sources: GOC:BHF, GOC:TermGenie, GOC:hal, GO_REF:0000067 Relationships: is a type of cation binding [GO:0043169]; is a type of sulfur compound binding [GO:1901681] Definition: Binding to S-adenosyl-L-methionine.